{
  "term_id": "GO:0008630",
  "gene": "UniProtKB:Q13315",
  "gene_name": "Serine-protein kinase ATM",
  "term_label": "intrinsic apoptotic signaling pathway in response to DNA damage",
  "gene_symbol": "ATM"
}